{
  "term_id": "GO:0005737",
  "gene_name": "Cytochrome P450 2A7",
  "gene_symbol": "CYP2A7",
  "gene": "UniProtKB:P20853",
  "term_label": "cytoplasm"
}